myosin VIII complex [GO:0031478] (cellular component) Relationships: is a type of unconventional myosin complex [GO:0016461] Definition: A myosin complex containing a dimer of class VIII myosin heavy chains and associated light chains. Myosin VIII is predicted to be dimeric, and contain an unusual 100-190 residue N-terminal extension prior to their motor domains, 3-4 IQ motifs, a short region (~70 residues) of predicted alpha-helical coiled coil and a C-terminal domain. References: PMID:25247701